{
  "term_id": "GO:0030016",
  "gene_symbol": "MYL9",
  "gene_name": "Myosin regulatory light polypeptide 9",
  "gene": "UniProtKB:P24844",
  "term_label": "myofibril"
}